cytochrome biosynthetic process [GO:1903605] (biological process) Also known as: cytochrome anabolism, cytochrome biosynthesis, cytochrome formation, cytochrome synthesis Subtypes: cytochrome c biosynthetic process [GO:1903607] Relationships: is a type of GO:0009059; is a type of cytochrome metabolic process [GO:1903604] References: PMID:19721088 Sources: GOC:TermGenie, GOC:dph, GO_REF:0000068 Definition: The chemical reactions and pathways resulting in the formation of a cytochrome.